{
  "gene_symbol": "CSF1R",
  "term_id": "GO:0008284",
  "term_label": "positive regulation of cell population proliferation",
  "gene": "UniProtKB:P07333",
  "gene_name": "Macrophage colony-stimulating factor 1 receptor"
}